mitochondria-associated endoplasmic reticulum membrane contact site [GO:0044233] (cellular component) Definition: A zone of apposition between endoplasmic-reticulum and mitochondrial membranes, structured by bridging complexes. These contact sites are thought to facilitate inter-organelle calcium and phospholipid exchange. Also known as: ER-mitochondrion membrane contact site, endoplasmic reticulum-mitochondrion membrane contact site, mitochondria-associated ER membrane, mitochondria-associated membrane, mitochondria-endoplasmic reticulum (ER) contact, MAM Relationships: is a type of GO:0044232 References: PMID:19556461, PMID:22078959, PMID:29626751, PMID:29684109 Sources: GOC:jl